{
  "gene_symbol": "TMEM107",
  "term_id": "UNKNOWN:0001",
  "term_label": "Unknown molecular function",
  "gene": "UniProtKB:Q6UX40",
  "gene_name": "Transmembrane protein 107"
}